quercetin 2,3-dioxygenase activity [GO:0008127] (molecular function) Also known as: flavonol 2,4-oxygenase activity, quercetin:oxygen 2,3-oxidoreductase (decyclizing), quercetinase activity Definition: Catalysis of the reaction: H+ + O2 + quercetin = 2-(3,4-dihydroxybenzoyloxy)-4,6-dihydroxybenzoate + CO. Sources: EC:1.13.11.24, RHEA:15381 Relationships: is_a oxidoreductase activity, acting on single donors with incorporation of molecular oxygen, incorporation of two atoms of oxygen [GO:0016702]